{
  "gene": "UniProtKB:O95159",
  "term_label": "Unknown biological process",
  "gene_name": "Zinc finger protein-like 1",
  "term_id": "UNKNOWN:0002",
  "gene_symbol": "ZFPL1"
}